{
  "gene_symbol": "ASCC1",
  "gene": "UniProtKB:Q8N9N2",
  "gene_name": "Activating signal cointegrator 1 complex subunit 1",
  "term_id": "GO:0006355",
  "term_label": "regulation of DNA-templated transcription"
}